cellular response to bacterial lipopeptide [GO:0071221] (biological process) Sources: GOC:mah Relationships: is a type of response to bacterial lipopeptide [GO:0070339]; is a type of cellular response to bacterial lipoprotein [GO:0071220] Definition: Any process that results in a change in state or activity of a cell (in terms of movement, secretion, enzyme production, gene expression, etc.) as a result of a bacterial lipopeptide stimulus. Subtypes: cellular response to diacyl bacterial lipopeptide [GO:0071726], cellular response to triacyl bacterial lipopeptide [GO:0071727]